{
  "gene_symbol": "PPP2R3C",
  "term_label": "cortical cytoskeleton organization",
  "gene_name": "Serine_threonine-protein phosphatase 2A regulatory subunit B'' subunit gamma",
  "gene": "UniProtKB:Q969Q6",
  "term_id": "GO:0030865"
}